{
  "term_label": "nuclear receptor-mediated steroid hormone signaling pathway",
  "gene_symbol": "PGR",
  "term_id": "GO:0030518",
  "gene": "UniProtKB:P06401",
  "gene_name": "Progesterone receptor"
}